{
  "gene_name": "Microtubule-associated protein RP_EB family member 3",
  "term_id": "GO:0035371",
  "term_label": "microtubule plus-end",
  "gene": "UniProtKB:Q9UPY8",
  "gene_symbol": "MAPRE3"
}